{
  "term_label": "serine-type endopeptidase activity",
  "gene": "UniProtKB:A6NIE9",
  "gene_name": "Putative serine protease 29",
  "gene_symbol": "PRSS29P",
  "term_id": "GO:0004252"
}